{
  "gene_name": "A-kinase anchor protein 13",
  "gene": "UniProtKB:Q12802",
  "term_label": "small GTPase-mediated signal transduction",
  "term_id": "GO:0007264",
  "gene_symbol": "AKAP13"
}